nuclear fragmentation involved in apoptotic nuclear change [GO:0030264] (biological process) Definition: The breakdown of the nucleus into small membrane-bounded compartments, or blebs, each of which contain compacted DNA. Also known as: apoptotic nuclear fragmentation, nucleus fragmentation, nuclear fragmentation during apoptosis Relationships: is a type of nuclear membrane organization [GO:0071763]; is part of GO:0030262 Sources: GOC:dph, GOC:mah, GOC:mtg_apoptosis, GOC:tb, ISBN:0721639976